{
  "gene_name": "T-cell-specific surface glycoprotein CD28",
  "gene_symbol": "CD28",
  "gene": "UniProtKB:P10747",
  "term_id": "GO:0042102",
  "term_label": "positive regulation of T cell proliferation"
}